regulation of hyphopodium formation [GO:0075188] (biological process) Note: Note that this term should not be used to annotate gene products of the host. It should only be used to annotate those gene products from the symbiont involved in this process. Subtypes: positive regulation of hyphopodium formation [GO:0075189], GO:0075190 Sources: GOC:pamgo_curators Also known as: regulation of hyphopodium formation on or near host Definition: Any process that modulates the frequency, rate or extent of symbiont hyphopodium formation on or near its host organism. The host is defined as the larger of the organisms involved in a symbiotic interaction. Relationships: is a type of regulation of anatomical structure morphogenesis [GO:0022603]; regulates hyphopodium formation [GO:0075187]